{
  "term_id": "GO:0050839",
  "gene_symbol": "PCDHA7",
  "term_label": "cell adhesion molecule binding",
  "gene_name": "Protocadherin alpha-7",
  "gene": "UniProtKB:Q9UN72"
}